negative regulation of pulmonary blood vessel remodeling [GO:1905110] (biological process) Relationships: is a type of negative regulation of blood vessel remodeling [GO:0060313]; is a type of GO:1905109; negatively regulates pulmonary blood vessel remodeling [GO:0101010] References: PMID:22161164 Sources: GOC:BHF, GOC:BHF_miRNA, GOC:TermGenie, GOC:bc, GO_REF:0000058 Definition: Any process that stops, prevents or reduces the frequency, rate or extent of pulmonary blood vessel remodeling. Also known as: down regulation of pulmonary blood vessel remodeling, down-regulation of pulmonary blood vessel remodeling, downregulation of pulmonary blood vessel remodeling, negative regulation of pulmonary blood vessel remodelling, inhibition of pulmonary blood vessel remodeling